animal organ morphogenesis [GO:0009887] (biological process) Subtypes: GO:0003007, imaginal disc morphogenesis [GO:0007560], chaeta morphogenesis [GO:0008407], GO:0022612, genitalia morphogenesis [GO:0035112], spermathecum morphogenesis [GO:0035211], gonad morphogenesis [GO:0035262], oviduct morphogenesis [GO:0035848], odontogenesis [GO:0042476], skin morphogenesis [GO:0043589], embryonic organ morphogenesis [GO:0048562], muscle organ morphogenesis [GO:0048644], skeletal system morphogenesis [GO:0048705], GO:0048734, GO:0048795, brain morphogenesis [GO:0048854], bone morphogenesis [GO:0060349], lung morphogenesis [GO:0060425], bronchus morphogenesis [GO:0060434], trachea morphogenesis [GO:0060439], cartilage morphogenesis [GO:0060536], kidney morphogenesis [GO:0060993], uterus morphogenesis [GO:0061038], pancreas morphogenesis [GO:0061113], GO:0072197, GO:0090596, nematode pharynx morphogenesis [GO:0110040], larynx morphogenesis [GO:0120223] Regulation: positively regulated by GO:0110110; negatively regulated by negative regulation of animal organ morphogenesis [GO:0110111]; regulated by regulation of animal organ morphogenesis [GO:2000027] Relationships: is a type of anatomical structure morphogenesis [GO:0009653]; is part of animal organ development [GO:0048513] Sources: GOC:dgh, GOC:go_curators, ISBN:0471245208, ISBN:0721662544 Definition: Morphogenesis of an animal organ. An organ is defined as a tissue or set of tissues that work together to perform a specific function or functions. Morphogenesis is the process in which anatomical structures are generated and organized. Organs are commonly observed as visibly distinct structures, but may also exist as loosely associated clusters of cells that work together to perform a specific function or functions. Also known as: histogenesis and organogenesis